{
  "term_id": "GO:0000981",
  "gene_symbol": "BARX2",
  "gene_name": "Homeobox protein BarH-like 2",
  "term_label": "DNA-binding transcription factor activity, RNA polymerase II-specific",
  "gene": "UniProtKB:Q9UMQ3"
}